{
  "gene": "UniProtKB:P01034",
  "term_id": "GO:0005737",
  "gene_name": "Cystatin-C",
  "gene_symbol": "CST3",
  "term_label": "cytoplasm"
}